{
  "term_id": "GO:0050660",
  "gene_name": "Acyl-coenzyme A oxidase-like protein",
  "gene_symbol": "ACOXL",
  "gene": "UniProtKB:Q9NUZ1",
  "term_label": "flavin adenine dinucleotide binding"
}